{
  "term_id": "GO:0034736",
  "gene": "UniProtKB:P35610",
  "term_label": "cholesterol O-acyltransferase activity",
  "gene_name": "Sterol O-acyltransferase 1",
  "gene_symbol": "SOAT1"
}